{
  "gene_name": "Transmembrane protein 151A",
  "term_label": "Unknown biological process",
  "term_id": "UNKNOWN:0002",
  "gene": "UniProtKB:Q8N4L1",
  "gene_symbol": "TMEM151A"
}